{
  "term_id": "GO:0008360",
  "gene": "UniProtKB:O95466",
  "gene_name": "Formin-like protein 1",
  "term_label": "regulation of cell shape",
  "gene_symbol": "FMNL1"
}